20-hydroxy-leukotriene B4 omega oxidase activity [GO:0097258] (molecular function) References: PMID:2836406, PMID:9675028 Sources: GOC:mw, RHEA:48668 Also known as: 20-hydroxy-leukotriene B4 omega-oxidase activity, 20-hydroxy-leukotriene B4 omega-oxidation Definition: Catalysis of the reaction: 20-hydroxy-leukotriene B4 + O2 + reduced [NADPH-hemoprotein reductase] = 20-oxo-leukotriene B4 + H+ + 2 H2O + oxidized [NADPH-hemoprotein reductase]. Relationships: is a type of monooxygenase activity [GO:0004497]; is a type of oxidoreductase activity, acting on CH-OH group of donors [GO:0016614]